{
  "term_label": "peptidyl-tRNA hydrolase activity",
  "gene_symbol": "MRPL58",
  "gene": "UniProtKB:Q14197",
  "gene_name": "Large ribosomal subunit protein mL62",
  "term_id": "GO:0004045"
}